{
  "gene_symbol": "MRPS10",
  "gene": "UniProtKB:P82664",
  "term_id": "UNKNOWN:0001",
  "term_label": "Unknown molecular function",
  "gene_name": "Small ribosomal subunit protein uS10m"
}